{
  "term_label": "regulation of gene expression",
  "gene_symbol": "TRIM6",
  "gene_name": "Tripartite motif-containing protein 6",
  "term_id": "GO:0010468",
  "gene": "UniProtKB:Q9C030"
}